{
  "gene": "UniProtKB:Q99558",
  "term_label": "Unknown molecular function",
  "gene_name": "Mitogen-activated protein kinase kinase kinase 14",
  "term_id": "UNKNOWN:0001",
  "gene_symbol": "MAP3K14"
}